{
  "term_id": "GO:0055088",
  "gene_symbol": "TLCD3B",
  "term_label": "lipid homeostasis",
  "gene_name": "Ceramide synthase",
  "gene": "UniProtKB:Q71RH2"
}